protein localization to endoplasmic reticulum [GO:0070972] (biological process) Regulation: regulated by regulation of protein localization to endoplasmic reticulum [GO:1905550]; negatively regulated by GO:1905551; positively regulated by positive regulation of protein localization to endoplasmic reticulum [GO:1905552] Sources: GOC:mah Definition: A process in which a protein is transported to, or maintained in, a location within the endoplasmic reticulum. Subtypes: protein localization to endoplasmic reticulum exit site [GO:0070973], protein localization to endoplasmic reticulum tubular network [GO:1903420] Relationships: is a type of GO:0033365 Also known as: protein localisation in endoplasmic reticulum, protein localization in ER, protein localization in endoplasmic reticulum